peptide antibiotic biosynthetic process [GO:0030651] (biological process) Also known as: peptide antibiotic anabolism, peptide antibiotic biosynthesis, peptide antibiotic formation, peptide antibiotic synthesis Relationships: is a type of GO:0017000; is a type of peptide biosynthetic process [GO:0043043]; is a type of amide biosynthetic process [GO:0043604] Subtypes: GO:0030152, GO:0033072 Definition: The chemical reactions and pathways resulting in the formation of peptides with antibiotic activity. Sources: GOC:mah